{
  "term_id": "GO:0001671",
  "gene_name": "Mitochondrial import inner membrane translocase subunit TIM14",
  "term_label": "ATPase activator activity",
  "gene_symbol": "DNAJC19",
  "gene": "UniProtKB:Q96DA6"
}